1-phosphatidylinositol binding [GO:0005545] (molecular function) Relationships: is_a phosphatidylinositol binding [GO:0035091] Sources: ISBN:0198506732 Definition: Binding to a phosphatidylinositol, a glycophospholipid with its sn-glycerol 3-phosphate residue is esterified to the 1-hydroxyl group of 1D-myo-inositol.